{
  "gene_symbol": "GPATCH3",
  "gene_name": "G patch domain-containing protein 3",
  "term_id": "UNKNOWN:0001",
  "gene": "UniProtKB:Q96I76",
  "term_label": "Unknown molecular function"
}